{
  "gene": "UniProtKB:Q8IWW8",
  "gene_symbol": "ADHFE1",
  "gene_name": "Hydroxyacid-oxoacid transhydrogenase, mitochondrial",
  "term_label": "mitochondrion",
  "term_id": "GO:0005739"
}